{
  "gene_symbol": "TOMM20",
  "gene": "UniProtKB:Q15388",
  "term_label": "mitochondrial outer membrane translocase complex",
  "gene_name": "Mitochondrial import receptor subunit TOM20 homolog",
  "term_id": "GO:0005742"
}